{
  "term_label": "cytosol",
  "gene_name": "Small ribosomal subunit protein RACK1",
  "gene": "UniProtKB:P63244",
  "term_id": "GO:0005829",
  "gene_symbol": "RACK1"
}